{
  "gene_name": "Protein-glutamine gamma-glutamyltransferase 4",
  "term_label": "protein-glutamine gamma-glutamyltransferase activity",
  "gene_symbol": "TGM4",
  "term_id": "GO:0003810",
  "gene": "UniProtKB:P49221"
}